intracellularly calcium-gated chloride channel activity [GO:0005229] (molecular function) Definition: Enables the transmembrane transfer of chloride by a channel that opens in response to stimulus by a calcium ion or ions. Transport by a channel involves catalysis of facilitated diffusion of a solute (by an energy-independent process) involving passage through a transmembrane aqueous pore or channel, without evidence for a carrier-mediated mechanism. Relationships: is a type of chloride channel activity [GO:0005254]; is a type of GO:0099095; is_a intracellularly calcium-gated channel activity [GO:0141147] References: PMID:29236691 Sources: GOC:mtg_transport Also known as: intracellular calcium activated chloride channel activity